{
  "term_label": "Unknown cellular component",
  "term_id": "UNKNOWN:0003",
  "gene_symbol": "CST6",
  "gene": "UniProtKB:Q15828",
  "gene_name": "Cystatin-M"
}